regulation of estrone secretion [GO:2000867] (biological process) Sources: GOC:sl Subtypes: GO:2000868, positive regulation of estrone secretion [GO:2000869] Also known as: regulation of 3-hydroxy-1,3,5(10)-estratrien-17-one secretion, regulation of folliculin secretion Definition: Any process that modulates the frequency, rate or extent of estrone secretion. Relationships: is a type of regulation of steroid hormone secretion [GO:2000831]; regulates GO:0035943